{
  "gene": "UniProtKB:Q9UGJ0",
  "gene_name": "5'-AMP-activated protein kinase subunit gamma-2",
  "term_label": "positive regulation of gluconeogenesis",
  "gene_symbol": "PRKAG2",
  "term_id": "GO:0045722"
}